{
  "term_id": "GO:1902115",
  "gene_symbol": "NF2",
  "gene_name": "Merlin",
  "term_label": "regulation of organelle assembly",
  "gene": "UniProtKB:P35240"
}